{
  "gene_symbol": "SDE2",
  "term_label": "Unknown molecular function",
  "gene": "UniProtKB:Q6IQ49",
  "term_id": "UNKNOWN:0001",
  "gene_name": "Splicing regulator SDE2"
}